{
  "gene": "UniProtKB:Q9ULT0",
  "gene_symbol": "TTC7A",
  "term_label": "protein localization to plasma membrane",
  "term_id": "GO:0072659",
  "gene_name": "Tetratricopeptide repeat protein 7A"
}